{
  "term_id": "GO:0005634",
  "gene_symbol": "ZNF488",
  "term_label": "nucleus",
  "gene": "UniProtKB:Q96MN9",
  "gene_name": "Zinc finger protein 488"
}